{
  "term_label": "piRNA binding",
  "gene_symbol": "PIWIL1",
  "term_id": "GO:0034584",
  "gene_name": "Piwi-like protein 1",
  "gene": "UniProtKB:Q96J94"
}